{
  "term_id": "GO:0006906",
  "gene_name": "Syntaxin-7",
  "term_label": "vesicle fusion",
  "gene": "UniProtKB:O15400",
  "gene_symbol": "STX7"
}